{
  "gene_name": "SMAD5 antisense gene protein 1",
  "gene_symbol": "SMAD5-AS1",
  "term_id": "UNKNOWN:0003",
  "gene": "UniProtKB:Q9Y6J3",
  "term_label": "Unknown cellular component"
}